N-acetylglucosamine kinase activity [GO:0045127] (MF) Sources: RHEA:17417 Definition: Catalysis of the reaction: N-acetyl-D-glucosamine + ATP = N-acetyl-D-glucosamine 6-phosphate + ADP + H+. Relationships: is a type of GO:0019200 Also known as: 2-acetylamino-2-deoxy-D-glucose kinase activity, ATP:2-acetylamino-2-deoxy-D-glucose 6-phosphotransferase activity, ATP:N-acetyl-D-glucosamine 6-phosphotransferase activity, GlcNAc kinase activity, acetylaminodeoxyglucokinase activity, acetylglucosamine kinase (phosphorylating)